{
  "gene_symbol": "KRTAP3-2",
  "gene": "UniProtKB:Q9BYR7",
  "term_label": "Unknown biological process",
  "term_id": "UNKNOWN:0002",
  "gene_name": "Keratin-associated protein 3-2"
}